{
  "gene_symbol": "MINAR1",
  "term_id": "UNKNOWN:0001",
  "gene": "UniProtKB:Q9UPX6",
  "gene_name": "Major intrinsically disordered Notch2-binding receptor 1",
  "term_label": "Unknown molecular function"
}